{
  "gene_name": "Microtubule-associated protein 1B",
  "gene": "UniProtKB:P46821",
  "term_label": "microtubule cytoskeleton organization",
  "term_id": "GO:0000226",
  "gene_symbol": "MAP1B"
}